positive regulation of cyclin-dependent protein serine/threonine kinase activity [GO:0045737] (biological process) Sources: GOC:go_curators, GOC:pr Definition: Any process that activates or increases the frequency, rate or extent of CDK activity. Relationships: is a type of regulation of cyclin-dependent protein serine/threonine kinase activity [GO:0000079]; is a type of positive regulation of cell cycle [GO:0045787]; is a type of positive regulation of protein serine/threonine kinase activity [GO:0071902]; is a type of GO:1904031; RO_0002213 cyclin-dependent protein serine/threonine kinase activity [GO:0004693] Also known as: activation of cyclin-dependent protein kinase activity, positive regulation of CDK activity, positive regulation of cyclin-dependent protein kinase activity, stimulation of cyclin-dependent protein kinase activity, up regulation of cyclin-dependent protein kinase activity, up-regulation of cyclin-dependent protein kinase activity, upregulation of cyclin-dependent protein kinase activity